{
  "gene_name": "T-cell leukemia translocation-altered gene protein",
  "term_id": "UNKNOWN:0003",
  "gene_symbol": "TCTA",
  "gene": "UniProtKB:P57738",
  "term_label": "Unknown cellular component"
}